{
  "gene_symbol": "AURKB",
  "term_label": "spindle midzone",
  "gene": "UniProtKB:Q96GD4",
  "term_id": "GO:0051233",
  "gene_name": "Aurora kinase B"
}